{
  "term_id": "GO:0050821",
  "term_label": "protein stabilization",
  "gene": "UniProtKB:Q9NX55",
  "gene_symbol": "HYPK",
  "gene_name": "Huntingtin-interacting protein K"
}